{
  "gene": "UniProtKB:Q9UBV4",
  "gene_name": "Protein Wnt-16",
  "term_label": "cell fate commitment",
  "gene_symbol": "WNT16",
  "term_id": "GO:0045165"
}